{
  "gene": "UniProtKB:Q6P1N9",
  "gene_symbol": "TATDN1",
  "term_label": "3'-5'-DNA exonuclease activity",
  "gene_name": "Deoxyribonuclease TATDN1",
  "term_id": "GO:0008296"
}